{
  "gene_symbol": "PBRM1",
  "term_label": "SWI/SNF complex",
  "term_id": "GO:0016514",
  "gene_name": "Protein polybromo-1",
  "gene": "UniProtKB:Q86U86"
}